lysophagy [GO:0062093] (biological process) Definition: The selective autophagy process in which a damaged lysosome is degraded by macroautophagy. Relationships: is a type of macroautophagy [GO:0016236] References: PMID:28743755